kanamycin catabolic process [GO:1901132] (biological process) Relationships: is a type of aminoglycoside antibiotic catabolic process [GO:0030649]; is a type of GO:0046174 Definition: The chemical reactions and pathways resulting in the breakdown of kanamycin. Sources: GOC:TermGenie, GOC:yaf, UniPathway:UPA00965 Also known as: kanamycin breakdown, kanamycin catabolism, kanamycin degradation